{
  "gene_symbol": "AKIRIN2",
  "term_label": "nucleus",
  "term_id": "GO:0005634",
  "gene": "UniProtKB:Q53H80",
  "gene_name": "Akirin-2"
}